{
  "gene": "UniProtKB:Q9UMX5",
  "gene_symbol": "NENF",
  "gene_name": "Neudesin",
  "term_id": "GO:0005783",
  "term_label": "endoplasmic reticulum"
}